positive regulation of pancreatic trypsinogen secretion [GO:1904244] (biological process) References: PMID:12771515 Sources: GOC:TermGenie, GO_REF:0000058 Definition: Any process that activates or increases the frequency, rate or extent of pancreatic trypsinogen secretion. Also known as: positive regulation of pancreatic trypsinogen release, up regulation of pancreatic trypsinogen release, up regulation of pancreatic trypsinogen secretion, up-regulation of pancreatic trypsinogen release, up-regulation of pancreatic trypsinogen secretion, upregulation of pancreatic trypsinogen release, upregulation of pancreatic trypsinogen secretion, activation of pancreatic trypsinogen release, activation of pancreatic trypsinogen secretion Relationships: is a type of positive regulation of protein secretion [GO:0050714]; is a type of regulation of pancreatic trypsinogen secretion [GO:1904242]; positively regulates GO:1990747